{
  "gene_name": "Kinesin-like protein KIF3A",
  "term_id": "GO:0060271",
  "term_label": "cilium assembly",
  "gene": "UniProtKB:Q9Y496",
  "gene_symbol": "KIF3A"
}